coronary sinus valve development [GO:0003178] (biological process) Definition: The progression of the valve of the coronary sinus over time, from its formation to the mature structure. Relationships: is a type of heart valve development [GO:0003170] Sources: GOC:mtg_heart